{
  "gene": "UniProtKB:Q5BIV9",
  "gene_name": "Shadow of prion protein",
  "gene_symbol": "SPRN",
  "term_label": "protein import into nucleus",
  "term_id": "GO:0006606"
}